chlorophyllase activity [GO:0047746] (molecular function) Sources: RHEA:19605 Also known as: chlorophyll chlorophyllidohydrolase activity Definition: Catalysis of the reaction: chlorophyll + H2O = phytol + chlorophyllide. Relationships: is_a carboxylic ester hydrolase activity [GO:0052689]